isotype switching to IgD isotypes [GO:0048292] (biological process) Note: Note that this term is to be used only for gene products involved in the expression of IgD through recombinational switching into the vestigial switch region at the 5' end of the IgD gene segment, rather than gene products involved in the expression of IgD through alternative splicing mechanisms. Also known as: class switching to IgD isotypes, isotype switch recombination to IgD isotypes Regulation: RO_0002211 by regulation of isotype switching to IgD isotypes [GO:0048299]; negatively regulated by GO:0048300; RO_0002213 by positive regulation of isotype switching to IgD isotypes [GO:0048301] Definition: The switching of activated B cells from IgM biosynthesis to IgD biosynthesis, accomplished through a recombination process involving an intrachromosomal deletion between switch regions that reside 5' of the IgM and IgD constant region gene segments in the immunoglobulin heavy chain locus. References: PMID:12370374, PMID:2113175, PMID:9186655 Sources: ISBN:0781735149 Relationships: is a type of isotype switching [GO:0045190]